tRNA (adenine(22)-N1)-methyltransferase activity [GO:0160105] (molecular function) Also known as: tRNA (adenine(22)-N(1))-methyltransferase activity, tRNA (adenosine(22)-N(1))-methyltransferase activity Definition: Catalysis of the reaction: adenosine(22) in tRNA + S-adenosyl-L-methionine = H+ + N(1)-methyladenosine(22) in tRNA + S-adenosyl-L-homocysteine. Relationships: is a type of tRNA (adenine) methyltransferase activity [GO:0016426] Sources: EC:2.1.1.217